{
  "term_label": "DNA-binding transcription factor activity, RNA polymerase II-specific",
  "gene_name": "Hypermethylated in cancer 1 protein",
  "gene": "UniProtKB:Q14526",
  "term_id": "GO:0000981",
  "gene_symbol": "HIC1"
}